nuclear migration involved in conjugation with mutual genetic exchange [GO:0000745] (biological process) Sources: GOC:clt, GOC:mah Relationships: is a type of nuclear migration [GO:0007097]; is part of GO:0000744 Definition: The net movement of nuclei towards one another, leading to the bilateral transfer of genetic material in organisms undergoing conjugation without cellular fusion. Also known as: nuclear migration involved in conjugation without cellular fusion, nuclear exchange during conjugation without cellular fusion